{
  "gene": "UniProtKB:Q9NZD2",
  "gene_name": "Glycolipid transfer protein",
  "term_id": "GO:0035627",
  "gene_symbol": "GLTP",
  "term_label": "ceramide transport"
}